{
  "term_id": "UNKNOWN:0002",
  "gene": "UniProtKB:Q8N2G6",
  "gene_symbol": "ZCCHC24",
  "gene_name": "Zinc finger CCHC domain-containing protein 24",
  "term_label": "Unknown biological process"
}